{
  "gene_symbol": "RBL2",
  "gene_name": "Retinoblastoma-like protein 2",
  "term_id": "GO:0000977",
  "term_label": "RNA polymerase II transcription regulatory region sequence-specific DNA binding",
  "gene": "UniProtKB:Q08999"
}